G protein-coupled receptor signaling pathway involved in heart process [GO:0086103] (BP) Also known as: G-protein coupled receptor signaling pathway involved in heart process, G-protein coupled receptor signalling pathway involved in heart process, GPCR signaling pathway involved in cardiac process, GPCR signaling pathway involved in heart process Subtypes: adenylate cyclase-activating adrenergic receptor signaling pathway involved in heart process [GO:0086023], G protein-coupled acetylcholine receptor signaling pathway involved in heart process [GO:0086093], GO:0086098, endothelin receptor signaling pathway involved in heart process [GO:0086101] Definition: An G protein-coupled receptor signaling pathway which contributes to a circulatory system process carried out by the heart. References: PMID:17376402 Sources: GOC:BHF, GOC:mtg_cardiac_conduct_nov11 Relationships: is a type of GO:0007186; is part of heart process [GO:0003015]